protein localization to nuclear inner membrane [GO:0036228] (biological process) Also known as: protein targeting to INM, protein targeting to nuclear inner membrane References: PMID:16929305 Sources: GOC:dgf Definition: A process in which a protein is transported to, or maintained in, a location within the nuclear inner membrane. Relationships: is a type of GO:0072657; is a type of protein localization to nuclear envelope [GO:0090435]